regulation of sensory neuron axon guidance [GO:1905489] (biological process) Relationships: is a type of regulation of axon guidance [GO:1902667]; regulates sensory neuron axon guidance [GO:0097374] Subtypes: negative regulation of sensory neuron axon guidance [GO:1905490], GO:1905491 Definition: Any process that modulates the frequency, rate or extent of sensory neuron axon guidance. References: PMID:16516839 Sources: GOC:TermGenie, GO_REF:0000058